{
  "gene": "UniProtKB:Q9H825",
  "gene_name": "tRNA N(3)-methylcytidine methyltransferase METTL8, mitochondrial",
  "gene_symbol": "METTL8",
  "term_id": "UNKNOWN:0003",
  "term_label": "Unknown cellular component"
}